{
  "gene_name": "Zinc finger protein 623",
  "term_id": "GO:0000978",
  "gene_symbol": "ZNF623",
  "gene": "UniProtKB:O75123",
  "term_label": "RNA polymerase II cis-regulatory region sequence-specific DNA binding"
}